{
  "term_label": "anatomical structure morphogenesis",
  "term_id": "GO:0009653",
  "gene_symbol": "PITX3",
  "gene_name": "Pituitary homeobox 3",
  "gene": "UniProtKB:O75364"
}